{
  "gene_symbol": "SSTR1",
  "term_id": "GO:0005886",
  "term_label": "plasma membrane",
  "gene": "UniProtKB:P30872",
  "gene_name": "Somatostatin receptor type 1"
}